{
  "term_label": "Unknown cellular component",
  "gene_name": "Leucine-rich repeat-containing protein 39",
  "gene_symbol": "LRRC39",
  "term_id": "UNKNOWN:0003",
  "gene": "UniProtKB:Q96DD0"
}